negative regulation of pinocytosis [GO:0048550] (biological process) Definition: Any process that stops, prevents, or reduces the frequency, rate or extent of pinocytosis. Pinocytosis is the process in which cells take in liquid material from their external environment; literally 'cell drinking'. Liquid is enclosed in vesicles, formed by invagination of the plasma membrane. These vesicles then move into the cell and pass their contents to endosomes. Sources: GOC:go_curators Also known as: down regulation of pinocytosis, down-regulation of pinocytosis, downregulation of pinocytosis, inhibition of pinocytosis Subtypes: negative regulation of macropinocytosis [GO:1905302] Relationships: is a type of negative regulation of endocytosis [GO:0045806]; is a type of GO:0048548; negatively regulates pinocytosis [GO:0006907]